{
  "term_id": "GO:0005634",
  "gene_symbol": "MBD3L2B",
  "gene": "UniProtKB:A0A1B0GVZ6",
  "term_label": "nucleus",
  "gene_name": "Methyl-CpG-binding domain protein 3-like 2B"
}